{
  "gene_name": "Sterol O-acyltransferase 1",
  "term_id": "GO:0008203",
  "gene_symbol": "SOAT1",
  "gene": "UniProtKB:P35610",
  "term_label": "cholesterol metabolic process"
}